positive regulation of cytoplasmic mRNA processing body assembly [GO:0010606] (biological process) Sources: GOC:dph, GOC:krc, GOC:tb Definition: Any process that increases the rate, frequency, or extent of the aggregation, arrangement and bonding together of proteins and RNA molecules to form a cytoplasmic mRNA processing body. Relationships: is a type of regulation of cytoplasmic mRNA processing body assembly [GO:0010603]; is a type of positive regulation of organelle assembly [GO:1902117]; positively regulates GO:0033962